{
  "gene": "UniProtKB:Q9H095",
  "gene_symbol": "IQCG",
  "term_id": "UNKNOWN:0001",
  "term_label": "Unknown molecular function",
  "gene_name": "Dynein regulatory complex protein 9"
}